{
  "term_label": "Unknown molecular function",
  "gene_name": "Protein FAM53A",
  "gene_symbol": "FAM53A",
  "term_id": "UNKNOWN:0001",
  "gene": "UniProtKB:Q6NSI3"
}